soyasapogenol B glucuronide galactosyltransferase activity [GO:0102240] (MF) Relationships: is a type of hexosyltransferase activity [GO:0016758] Definition: Catalysis of the reaction: UDP-D-galactose + soyasapogenol B 3-O-beta-glucuronate = H+ + UDP + soyasaponin III. Sources: EC:2.4.1.272, GOC:pz